oxidoreductase activity, acting on the CH-NH group of donors, iron-sulfur protein as acceptor [GO:0033694] (molecular function) Subtypes: methylenetetrahydrofolate reductase (ferredoxin) activity [GO:0033738] Sources: GOC:jl Relationships: is a type of oxidoreductase activity, acting on the CH-NH group of donors [GO:0016645] Definition: Catalysis of an oxidation-reduction (redox) reaction in which a CH-NH group acts as a hydrogen or electron donor and reduces an iron-sulfur protein.